{
  "term_label": "Unknown cellular component",
  "gene_symbol": "SHISAL2A",
  "term_id": "UNKNOWN:0003",
  "gene_name": "Protein shisa-like-2A",
  "gene": "UniProtKB:Q6UWV7"
}